{
  "gene_symbol": "SEPTIN8",
  "term_id": "GO:0003924",
  "gene": "UniProtKB:Q92599",
  "gene_name": "Septin-8",
  "term_label": "GTPase activity"
}